amitosis [GO:0051337] (biological process) Definition: Nuclear division that occurs by simple constriction of the nucleus without chromosome condensation or spindle formation. Sources: GOC:curators, ISBN:0721662544 Also known as: Remak nuclear division, direct nuclear division Relationships: is_a nuclear division [GO:0000280]